{
  "gene_symbol": "PCK1",
  "term_label": "manganese ion binding",
  "gene": "UniProtKB:P35558",
  "gene_name": "Phosphoenolpyruvate carboxykinase, cytosolic [GTP]",
  "term_id": "GO:0030145"
}